{
  "gene_name": "Threonine--tRNA ligase 1, cytoplasmic",
  "gene": "UniProtKB:P26639",
  "term_id": "GO:0006435",
  "term_label": "threonyl-tRNA aminoacylation",
  "gene_symbol": "TARS1"
}